transcription by RNA polymerase IV [GO:0001059] (biological process) Relationships: is_a DNA-templated transcription [GO:0006351] Also known as: transcription from RNA pol IV promoter, transcription from RNA polymerase IV promoter References: PMID:19110459 Sources: GOC:txnOH Definition: The synthesis of RNA from a DNA template by RNA polymerase IV, originating at a Pol IV-specific promoter.